{
  "term_id": "GO:0000379",
  "gene": "UniProtKB:Q9BSV6",
  "gene_symbol": "TSEN34",
  "term_label": "tRNA-type intron splice site recognition and cleavage",
  "gene_name": "tRNA-splicing endonuclease subunit Sen34"
}